{
  "term_id": "GO:0000981",
  "term_label": "DNA-binding transcription factor activity, RNA polymerase II-specific",
  "gene_symbol": "ZNF320",
  "gene_name": "Zinc finger protein 320",
  "gene": "UniProtKB:A2RRD8"
}